{
  "term_label": "Unknown molecular function",
  "gene_symbol": "NDUFA3",
  "term_id": "UNKNOWN:0001",
  "gene": "UniProtKB:O95167",
  "gene_name": "NADH dehydrogenase [ubiquinone] 1 alpha subcomplex subunit 3"
}